{
  "term_id": "UNKNOWN:0001",
  "gene": "UniProtKB:Q9UJW0",
  "gene_symbol": "DCTN4",
  "gene_name": "Dynactin subunit 4",
  "term_label": "Unknown molecular function"
}